{
  "gene_symbol": "NRL",
  "term_label": "retinal rod cell development",
  "gene_name": "Neural retina-specific leucine zipper protein",
  "term_id": "GO:0046548",
  "gene": "UniProtKB:P54845"
}